4-alpha-methyl-delta7-sterol oxidation [GO:0080065] (biological process) Relationships: is_a lipid oxidation [GO:0034440] Definition: A lipid oxidation process proceeding through a series of three successive monooxygenations of the alpha methyl group on the C4 carbon (CH3 to CH2OH to CHO to COOH) and resulting in this overall reaction: 4-alpha-methyl-delta7-sterol + 3 NADPH + 3 H+ + 3 O2 = 4-alpha-carboxy,delta7-sterol + 3 NADP+ + 3 H2O. Also known as: 4-alpha-methyl-delta7-sterol-4alpha-methyl oxidase activity References: PMID:14653780 Sources: GOC:pr